{
  "gene": "UniProtKB:Q6PGN9",
  "term_label": "spindle microtubule",
  "gene_symbol": "PSRC1",
  "gene_name": "Proline_serine-rich coiled-coil protein 1",
  "term_id": "GO:0005876"
}